{
  "gene_symbol": "OR10G4",
  "gene": "UniProtKB:Q8NGN3",
  "term_id": "GO:0004984",
  "term_label": "olfactory receptor activity",
  "gene_name": "Olfactory receptor 10G4"
}